{
  "term_label": "ubiquitin-dependent protein catabolic process",
  "gene_name": "E3 ubiquitin-protein ligase RNF13",
  "gene_symbol": "RNF13",
  "gene": "UniProtKB:O43567",
  "term_id": "GO:0006511"
}